{
  "gene_name": "Mitochondrial import inner membrane translocase subunit TIM50",
  "gene_symbol": "TIMM50",
  "term_label": "protein import into mitochondrial matrix",
  "term_id": "GO:0030150",
  "gene": "UniProtKB:Q3ZCQ8"
}